{
  "gene_name": "Gamma-aminobutyric acid receptor subunit alpha-4",
  "term_label": "postsynapse",
  "gene": "UniProtKB:P48169",
  "term_id": "GO:0098794",
  "gene_symbol": "GABRA4"
}